{
  "gene": "UniProtKB:P49418",
  "gene_name": "Amphiphysin",
  "term_label": "synaptic vesicle endocytosis",
  "term_id": "GO:0048488",
  "gene_symbol": "AMPH"
}